{
  "gene": "UniProtKB:Q8NA03",
  "gene_symbol": "FSIP1",
  "term_label": "Unknown cellular component",
  "term_id": "UNKNOWN:0003",
  "gene_name": "Fibrous sheath-interacting protein 1"
}